{
  "gene_symbol": "IGHG2",
  "term_id": "GO:0034987",
  "gene_name": "Immunoglobulin heavy constant gamma 2",
  "term_label": "immunoglobulin receptor binding",
  "gene": "UniProtKB:P01859"
}